negative regulation of netrin-activated signaling pathway [GO:1902842] (biological process) Also known as: down regulation of netrin signaling pathway, down regulation of netrin-activated signal transduction pathway, down regulation of netrin-activated signaling pathway, down regulation of netrin-activated signalling pathway, down regulation of netrin-mediated signaling pathway, down-regulation of netrin signaling pathway, down-regulation of netrin-activated signal transduction pathway, down-regulation of netrin-activated signaling pathway, down-regulation of netrin-activated signalling pathway, down-regulation of netrin-mediated signaling pathway, downregulation of netrin signaling pathway, downregulation of netrin-activated signal transduction pathway, downregulation of netrin-activated signaling pathway, downregulation of netrin-activated signalling pathway, downregulation of netrin-mediated signaling pathway, negative regulation of netrin signaling pathway, negative regulation of netrin-activated signal transduction pathway, negative regulation of netrin-activated signalling pathway, negative regulation of netrin-mediated signaling pathway, inhibition of netrin signaling pathway, inhibition of netrin-activated signal transduction pathway, inhibition of netrin-activated signaling pathway, inhibition of netrin-activated signalling pathway, inhibition of netrin-mediated signaling pathway References: PMID:24004945 Sources: GOC:TermGenie, GOC:kmv, GO_REF:0000058 Definition: Any process that stops, prevents or reduces the frequency, rate or extent of netrin-activated signaling pathway. Relationships: is_a negative regulation of signal transduction [GO:0009968]; is a type of regulation of netrin-activated signaling pathway [GO:1902841]; negatively regulates netrin-activated signaling pathway [GO:0038007]